{
  "gene_symbol": "SH2D4A",
  "gene": "UniProtKB:Q9H788",
  "term_id": "UNKNOWN:0002",
  "gene_name": "SH2 domain-containing protein 4A",
  "term_label": "Unknown biological process"
}